{
  "term_id": "GO:1902902",
  "term_label": "negative regulation of autophagosome assembly",
  "gene_symbol": "PHF23",
  "gene": "UniProtKB:Q9BUL5",
  "gene_name": "PHD finger protein 23"
}